{
  "term_label": "posterior lateral line neuromast hair cell development",
  "gene_name": "Transmembrane protein 132E",
  "term_id": "GO:0035677",
  "gene": "UniProtKB:Q6IEE7",
  "gene_symbol": "TMEM132E"
}